{
  "term_label": "plasma membrane",
  "gene": "UniProtKB:P16157",
  "gene_symbol": "ANK1",
  "gene_name": "Ankyrin-1",
  "term_id": "GO:0005886"
}